regulation of isotype switching to IgD isotypes [GO:0048299] (biological process) Sources: GOC:jid Relationships: is a type of regulation of isotype switching [GO:0045191]; regulates isotype switching to IgD isotypes [GO:0048292] Definition: Any process that modulates the frequency, rate or extent of isotype switching to IgD isotypes. Also known as: regulation of class switch recombination to IgD isotypes, regulation of class switching to IgD isotypes, regulation of isotype switch recombination to IgD isotypes Subtypes: GO:0048300, positive regulation of isotype switching to IgD isotypes [GO:0048301]